{
  "gene_symbol": "PPP1R9A",
  "term_label": "actin filament organization",
  "gene_name": "Neurabin-1",
  "gene": "UniProtKB:Q9ULJ8",
  "term_id": "GO:0007015"
}